{
  "gene_name": "Killer cell lectin-like receptor subfamily F member 2",
  "gene_symbol": "KLRF2",
  "gene": "UniProtKB:D3W0D1",
  "term_label": "plasma membrane",
  "term_id": "GO:0005886"
}